DNA-binding transcription activator activity [GO:0001216] (molecular function) Subtypes: DNA-binding transcription activator activity, RNA polymerase II-specific [GO:0001228], ligand-modulated transcription activator activity [GO:0141097] Also known as: bacterial-type RNA polymerase transcriptional activator activity, metal ion regulated sequence-specific DNA binding, bacterial-type RNA polymerase transcriptional activator activity, sequence-specific DNA binding, metal ion regulated sequence-specific DNA binding bacterial-type RNA polymerase transcription factor activity involved in positive regulation of transcription, sequence-specific DNA binding bacterial-type RNA polymerase transcription factor activity involved in positive regulation of transcription, transcriptional activator activity, bacterial-type RNA polymerase core promoter proximal region sequence-specific binding, bacterial-type RNA polymerase core promoter proximal region sequence-specific DNA binding transcription factor activity involved in positive regulation of transcription, transcriptional activator activity, bacterial-type RNA polymerase proximal promoter sequence-specific DNA binding Note: For usage guidance, see comment in GO:0003700 ; DNA-binding transcription factor activity. Sources: GOC:txnOH-2018 Relationships: is a type of DNA-binding transcription factor activity [GO:0003700]; is part of positive regulation of DNA-templated transcription [GO:0045893] Definition: A DNA-binding transcription factor activity that activates or increases transcription of specific gene sets.